{
  "gene_symbol": "WTIP",
  "term_label": "cytoskeleton organization",
  "gene_name": "Wilms tumor protein 1-interacting protein",
  "gene": "UniProtKB:A6NIX2",
  "term_id": "GO:0007010"
}